{
  "term_id": "GO:0042981",
  "gene_symbol": "USP17L8",
  "term_label": "regulation of apoptotic process",
  "gene_name": "Inactive ubiquitin carboxyl-terminal hydrolase 17-like protein 8",
  "gene": "UniProtKB:P0C7I0"
}